{
  "gene": "UniProtKB:Q9Y5R4",
  "gene_name": "MTRF1L release factor glutamine methyltransferase",
  "term_id": "UNKNOWN:0003",
  "gene_symbol": "HEMK1",
  "term_label": "Unknown cellular component"
}